{
  "term_label": "Unknown biological process",
  "term_id": "UNKNOWN:0002",
  "gene_symbol": "SMPX",
  "gene_name": "Small muscular protein",
  "gene": "UniProtKB:Q9UHP9"
}